{
  "gene": "UniProtKB:Q15825",
  "term_id": "GO:0051899",
  "term_label": "membrane depolarization",
  "gene_symbol": "CHRNA6",
  "gene_name": "Neuronal acetylcholine receptor subunit alpha-6"
}